{
  "term_id": "GO:0007155",
  "term_label": "cell adhesion",
  "gene": "UniProtKB:A6NMB1",
  "gene_symbol": "SIGLEC16",
  "gene_name": "Sialic acid-binding Ig-like lectin 16"
}